{
  "gene": "UniProtKB:Q9Y5P2",
  "term_id": "UNKNOWN:0003",
  "term_label": "Unknown cellular component",
  "gene_symbol": "CSAG3",
  "gene_name": "Chondrosarcoma-associated gene 2_3 protein"
}